{
  "gene": "UniProtKB:Q86T03",
  "gene_symbol": "PIP4P1",
  "gene_name": "Type 1 phosphatidylinositol 4,5-bisphosphate 4-phosphatase",
  "term_label": "plasma membrane",
  "term_id": "GO:0005886"
}